myosin V complex [GO:0031475] (cellular component) Sources: Wikipedia:Myosin Definition: A myosin complex containing a dimer of class V myosin heavy chains and associated light chains; involved in intracellular transport. Myosin V is a dimeric molecule consisting of conserved motor domains followed by 6 IQ motifs which bind specific light chains and calmodulin. The tail domain is important for cellular localization and cargo binding and can be divided into an alpha-helical coiled coil region and a C-terminal globular region. Relationships: is a type of GO:0016461